{
  "gene": "UniProtKB:Q9BZS1",
  "term_id": "GO:0001227",
  "gene_name": "Forkhead box protein P3",
  "term_label": "DNA-binding transcription repressor activity, RNA polymerase II-specific",
  "gene_symbol": "FOXP3"
}